{
  "term_label": "cytoplasm",
  "gene_symbol": "ACRV1",
  "gene_name": "Acrosomal protein SP-10",
  "gene": "UniProtKB:P26436",
  "term_id": "GO:0005737"
}